cytoplasmic helical capsid assembly [GO:0039711] (biological process) Relationships: is a type of cytoplasmic capsid assembly [GO:0039709] Definition: The assembly of a helical viral capsid in the cytoplasm. Occurs by assembling around the viral genome. Sources: VZ:1950